{
  "gene_symbol": "LRTM2",
  "term_label": "Unknown cellular component",
  "gene": "UniProtKB:Q8N967",
  "term_id": "UNKNOWN:0003",
  "gene_name": "Leucine-rich repeat and transmembrane domain-containing protein 2"
}